filamentous growth of a population of unicellular organisms in response to chemical stimulus [GO:0036171] (biological process) Regulation: regulated by regulation of filamentous growth of a population of unicellular organisms in response to chemical stimulus [GO:1900437]; negatively regulated by negative regulation of filamentous growth of a population of unicellular organisms in response to chemical stimulus [GO:1900438]; positively regulated by GO:1900439 References: PMID:17554048 Sources: GOC:di Definition: The process in which a group of unicellular organisms grow in a threadlike, filamentous shape in response to a chemical stimulus. Relationships: is_a filamentous growth of a population of unicellular organisms [GO:0044182]; is part of GO:0042221